{
  "gene_name": "Rac GTPase-activating protein 1",
  "gene_symbol": "RACGAP1",
  "term_id": "GO:0097149",
  "term_label": "centralspindlin complex",
  "gene": "UniProtKB:Q9H0H5"
}